{
  "gene_symbol": "TRIM9",
  "term_id": "UNKNOWN:0001",
  "term_label": "Unknown molecular function",
  "gene": "UniProtKB:Q9C026",
  "gene_name": "E3 ubiquitin-protein ligase TRIM9"
}